positive regulation of macrophage colony-stimulating factor signaling pathway [GO:1902228] (biological process) Also known as: positive regulation of M-CSF signaling pathway, positive regulation of macrophage colony-stimulating factor signalling pathway, up regulation of M-CSF signaling pathway, up regulation of macrophage colony-stimulating factor signaling pathway, up regulation of macrophage colony-stimulating factor signalling pathway, up-regulation of M-CSF signaling pathway, up-regulation of macrophage colony-stimulating factor signaling pathway, up-regulation of macrophage colony-stimulating factor signalling pathway, upregulation of M-CSF signaling pathway, upregulation of macrophage colony-stimulating factor signaling pathway, upregulation of macrophage colony-stimulating factor signalling pathway, activation of M-CSF signaling pathway, activation of macrophage colony-stimulating factor signaling pathway, activation of macrophage colony-stimulating factor signalling pathway References: PMID:16705167 Sources: GOC:TermGenie Definition: Any process that activates or increases the frequency, rate or extent of macrophage colony-stimulating factor signaling pathway. Relationships: is a type of positive regulation of cytokine-mediated signaling pathway [GO:0001961]; is a type of regulation of macrophage colony-stimulating factor signaling pathway [GO:1902226]; RO_0002213 macrophage colony-stimulating factor signaling pathway [GO:0038145]